regulation of D-xylose catabolic process [GO:0043469] (biological process) Relationships: is a type of regulation of carbohydrate catabolic process [GO:0043470]; is a type of regulation of small molecule metabolic process [GO:0062012]; regulates D-xylose catabolic process [GO:0042843] Definition: Any process that modulates the frequency, rate, or extent of the chemical reactions and pathways resulting in the breakdown of xylose. Subtypes: regulation of xylose catabolic process to ethanol [GO:1900515] Sources: GOC:mlg